{
  "gene_symbol": "SPATA2",
  "gene": "UniProtKB:Q9UM82",
  "term_id": "GO:0005737",
  "gene_name": "Spermatogenesis-associated protein 2",
  "term_label": "cytoplasm"
}